mitotic telomere clustering and tethering at nuclear periphery [GO:0120109] (biological process) References: PMID:25778919 Relationships: is a type of telomere localization [GO:0034397] Definition: The process in which the telomeres are gathered together to a small number of foci per chromosome (usually one per chromosome or fewer), and moved to and tethered at the nuclear periphery, as part of a mitotic cell cycle.